{
  "gene_symbol": "POMT2",
  "gene": "UniProtKB:Q9UKY4",
  "term_id": "GO:0005783",
  "gene_name": "Protein O-mannosyl-transferase 2",
  "term_label": "endoplasmic reticulum"
}